{
  "gene_name": "Zinc-activated ligand-gated ion channel",
  "gene_symbol": "ZACN",
  "term_label": "plasma membrane",
  "term_id": "GO:0005886",
  "gene": "UniProtKB:Q401N2"
}